{
  "term_label": "Unknown molecular function",
  "gene_name": "Vacuolar protein sorting-associated protein 51 homolog",
  "gene": "UniProtKB:Q9UID3",
  "gene_symbol": "VPS51",
  "term_id": "UNKNOWN:0001"
}